{
  "gene": "UniProtKB:Q92911",
  "term_label": "sodium ion transport",
  "gene_name": "Sodium_iodide cotransporter",
  "term_id": "GO:0006814",
  "gene_symbol": "SLC5A5"
}